{
  "term_label": "nucleus",
  "gene_name": "Putative spermatid-specific linker histone H1-like protein",
  "term_id": "GO:0005634",
  "gene_symbol": "H1-9P",
  "gene": "UniProtKB:P60008"
}